regulation of response to endoplasmic reticulum stress [GO:1905897] (biological process) Subtypes: GO:0060734, GO:1900101, GO:1902235, negative regulation of response to endoplasmic reticulum stress [GO:1903573], regulation of ERAD pathway [GO:1904292], positive regulation of response to endoplasmic reticulum stress [GO:1905898] References: PMID:21803450 Sources: GOC:TermGenie, GOC:aruk, GOC:bc, GO_REF:0000058 Relationships: is a type of regulation of cellular response to stress [GO:0080135]; regulates response to endoplasmic reticulum stress [GO:0034976] Also known as: regulation of ER stress response, regulation of cellular response to endoplasmic reticulum stress, regulation of response to ER stress Definition: Any process that modulates the frequency, rate or extent of response to endoplasmic reticulum stress.